{
  "gene_name": "Poly(rC)-binding protein 2",
  "gene": "UniProtKB:Q15366",
  "gene_symbol": "PCBP2",
  "term_label": "nucleoplasm",
  "term_id": "GO:0005654"
}